{
  "term_id": "GO:0030246",
  "gene_symbol": "CLEC4C",
  "gene": "UniProtKB:Q8WTT0",
  "gene_name": "C-type lectin domain family 4 member C",
  "term_label": "carbohydrate binding"
}